{
  "gene_symbol": "UBE2L6",
  "gene": "UniProtKB:O14933",
  "gene_name": "Ubiquitin_ISG15-conjugating enzyme E2 L6",
  "term_id": "GO:0000209",
  "term_label": "protein polyubiquitination"
}